spermatogonial cell division [GO:0007284] (biological process) Note: See also the Cell Ontology terms 'spermatogonium ; CL:0000020' and 'primary spermatocyte ; CL:0000656'. Relationships: is a type of cell division [GO:0051301]; is part of GO:0007283 Sources: GOC:bf, GOC:pr, ISBN:0879694238 Definition: The mitotic divisions of the primary spermatogonial cell (a primordial male germ cell) to form secondary spermatogonia (primary spermatocytes). Also known as: spermatogonium division